{
  "gene": "UniProtKB:Q15329",
  "term_label": "DNA-binding transcription factor activity, RNA polymerase II-specific",
  "gene_symbol": "E2F5",
  "term_id": "GO:0000981",
  "gene_name": "Transcription factor E2F5"
}